{
  "term_id": "GO:0009913",
  "gene_symbol": "OVOL1",
  "gene_name": "Putative transcription factor Ovo-like 1",
  "term_label": "epidermal cell differentiation",
  "gene": "UniProtKB:O14753"
}